{
  "gene": "UniProtKB:Q7RTS7",
  "term_label": "keratin filament",
  "gene_symbol": "KRT74",
  "gene_name": "Keratin, type II cytoskeletal 74",
  "term_id": "GO:0045095"
}